{
  "term_id": "GO:0031514",
  "gene": "UniProtKB:Q5H913",
  "gene_name": "ADP-ribosylation factor-like protein 13A",
  "term_label": "motile cilium",
  "gene_symbol": "ARL13A"
}